{
  "term_id": "GO:0035591",
  "term_label": "signaling adaptor activity",
  "gene": "UniProtKB:Q9NYB9",
  "gene_name": "Abl interactor 2",
  "gene_symbol": "ABI2"
}